regulation of chromosome separation [GO:1905818] (biological process) Subtypes: regulation of mitotic sister chromatid separation [GO:0010965], regulation of meiotic chromosome separation [GO:1905132], GO:1905819, positive regulation of chromosome separation [GO:1905820] References: PMID:21795393 Sources: GOC:TermGenie, GOC:bhm, GO_REF:0000058 Also known as: regulation of rDNA separation, regulation of chromatid release Definition: Any process that modulates the frequency, rate or extent of chromosome separation. Relationships: is a type of regulation of chromosome segregation [GO:0051983]; regulates GO:0051304